{
  "gene_symbol": "COLEC11",
  "gene_name": "Collectin-11",
  "term_label": "extracellular space",
  "gene": "UniProtKB:Q9BWP8",
  "term_id": "GO:0005615"
}